{
  "term_id": "GO:0030154",
  "gene_name": "Forkhead box protein D1",
  "gene_symbol": "FOXD1",
  "gene": "UniProtKB:Q16676",
  "term_label": "cell differentiation"
}